maltose alpha-D-glucosyltransferase activity [GO:0047471] (molecular function) Also known as: maltose alpha-D-glucosylmutase activity, maltose glucosylmutase activity, trehalose synthase activity Relationships: is a type of intramolecular transferase activity [GO:0016866] Definition: Catalysis of the reaction: maltose = trehalose. Sources: EC:5.4.99.16, MetaCyc:5.4.99.16-RXN